{
  "gene_name": "UNC5C-like protein",
  "gene_symbol": "UNC5CL",
  "term_label": "positive regulation of JNK cascade",
  "term_id": "GO:0046330",
  "gene": "UniProtKB:Q8IV45"
}